{
  "term_label": "regulation of actin cytoskeleton organization",
  "gene_symbol": "CIT",
  "gene_name": "Citron Rho-interacting kinase",
  "gene": "UniProtKB:O14578",
  "term_id": "GO:0032956"
}